{
  "term_id": "GO:0047023",
  "gene_name": "Aldo-keto reductase family 1 member C3",
  "gene": "UniProtKB:P42330",
  "term_label": "androsterone dehydrogenase [NAD(P)+] activity",
  "gene_symbol": "AKR1C3"
}